{
  "term_id": "GO:0005737",
  "term_label": "cytoplasm",
  "gene": "UniProtKB:Q9BZH6",
  "gene_symbol": "WDR11",
  "gene_name": "WD repeat-containing protein 11"
}